imaginal disc-derived appendage morphogenesis [GO:0035114] (biological process) Definition: The process in which the anatomical structures of appendages are generated and organized. An appendage is an organ or part that is attached to the trunk of an organism. Sources: GOC:mtg_sensu, ISBN:0582227089 Relationships: is a type of appendage morphogenesis [GO:0035107]; is part of imaginal disc-derived appendage development [GO:0048737] Subtypes: antennal development [GO:0007469], imaginal disc-derived wing morphogenesis [GO:0007476], imaginal disc-derived leg morphogenesis [GO:0007480], haltere morphogenesis [GO:0048735]